{
  "term_id": "GO:0005769",
  "term_label": "early endosome",
  "gene": "UniProtKB:O14964",
  "gene_symbol": "HGS",
  "gene_name": "Hepatocyte growth factor-regulated tyrosine kinase substrate"
}